{
  "term_id": "GO:0070934",
  "term_label": "CRD-mediated mRNA stabilization",
  "gene_name": "Insulin-like growth factor 2 mRNA-binding protein 2",
  "gene": "UniProtKB:Q9Y6M1",
  "gene_symbol": "IGF2BP2"
}